{
  "gene_symbol": "ETV7",
  "gene_name": "Transcription factor ETV7",
  "term_label": "DNA-binding transcription factor activity, RNA polymerase II-specific",
  "gene": "UniProtKB:Q9Y603",
  "term_id": "GO:0000981"
}